deubiquitinase activity [GO:0101005] (molecular function) Relationships: is a type of GO:0019783 Definition: An isopeptidase activity that cleaves ubiquitin from a target protein to which it is conjugated. References: PMID:30783221 Sources: GOC:mec Regulation: positively regulated by deubiquitinase activator activity [GO:0035800] Subtypes: cysteine-type deubiquitinase activity [GO:0004843], K63-linked deubiquitinase activity [GO:0061578], GO:0140492, histone deubiquitinase activity [GO:0140934], K11-linked deubiquitinase activity [GO:0180017], K48-linked deubiquitinase activity [GO:1990380] Note: There are two main classes of deubiquitinating enzymes: cysteine proteases (i.e., thiol dependent) and metalloproteases. Also known as: ubiquitinyl hydrolase activity